{
  "term_id": "GO:0099509",
  "gene": "UniProtKB:Q7L1I2",
  "term_label": "regulation of presynaptic cytosolic calcium ion concentration",
  "gene_symbol": "SV2B",
  "gene_name": "Synaptic vesicle glycoprotein 2B"
}